positive regulation of tolerance induction to self antigen [GO:0002651] (biological process) Definition: Any process that activates or increases the frequency, rate, or extent of tolerance induction to self antigen. Sources: GOC:add Also known as: up regulation of tolerance induction to self antigen, up-regulation of tolerance induction to self antigen, upregulation of tolerance induction to self antigen, activation of tolerance induction to self antigen, stimulation of tolerance induction to self antigen Relationships: is a type of positive regulation of tolerance induction [GO:0002645]; is a type of regulation of tolerance induction to self antigen [GO:0002649]; positively regulates tolerance induction to self antigen [GO:0002513]